positive regulation of protein K48-linked ubiquitination [GO:1902524] (biological process) References: PMID:21931591 Sources: GOC:TermGenie Definition: Any process that activates or increases the frequency, rate or extent of protein K48-linked ubiquitination. Note: An example is BIRC2 (UniProt ID Q13490) in PMID:21931591. Relationships: is a type of regulation of protein K48-linked ubiquitination [GO:0061945]; is a type of GO:1902916; RO_0002213 protein K48-linked ubiquitination [GO:0070936] Also known as: positive regulation of protein K48-linked polyubiquitination, up regulation of protein K48-linked polyubiquitination, up regulation of protein K48-linked ubiquitination, up-regulation of protein K48-linked polyubiquitination, up-regulation of protein K48-linked ubiquitination, upregulation of protein K48-linked polyubiquitination, upregulation of protein K48-linked ubiquitination, activation of protein K48-linked polyubiquitination, activation of protein K48-linked ubiquitination